{
  "term_id": "GO:0051010",
  "gene": "UniProtKB:Q9UDT6",
  "gene_name": "CAP-Gly domain-containing linker protein 2",
  "gene_symbol": "CLIP2",
  "term_label": "microtubule plus-end binding"
}